{
  "gene_name": "Protocadherin gamma-C5",
  "gene_symbol": "PCDHGC5",
  "gene": "UniProtKB:Q9Y5F6",
  "term_id": "GO:0050839",
  "term_label": "cell adhesion molecule binding"
}